cellulose catabolism by endo-processive cellulases [GO:0052785] (biological process) References: PMID:18035374 Sources: GOC:mengo_curators Definition: The breakdown into simpler components of cellulose. Catabolism is initiated by endohydrolytic attacks on the cellulose chain, and the resulting pieces are further degraded by cellulase enzymes to produce smaller and smaller fragments. Also known as: endo-processive cellulase activity Relationships: is a type of cellulose catabolic process [GO:0030245]